type I interferon-mediated signaling pathway [GO:0060337] (biological process) Relationships: is a type of GO:0140888; is part of GO:0071357 References: PMID:32464097 Sources: GOC:add, GOC:dph, GOC:signaling Also known as: type I interferon signaling pathway, type I interferon-activated signaling pathway Regulation: regulated by regulation of type I interferon-mediated signaling pathway [GO:0060338]; RO_0002212 by GO:0060339; positively regulated by positive regulation of type I interferon-mediated signaling pathway [GO:0060340] Definition: The series of molecular signals initiated by type I interferon binding to its receptor on the surface of a target cell, and ending with the regulation of a downstream cellular process, e.g. transcription. Type I interferons include the interferon-alpha, beta, delta, episilon, zeta, kappa, tau, and omega gene families.